{
  "term_label": "Unknown cellular component",
  "gene": "UniProtKB:P0C7X1",
  "term_id": "UNKNOWN:0003",
  "gene_symbol": "TBC1D3H",
  "gene_name": "TBC1 domain family member 3H"
}